N-acetylglucosaminyldiphosphodolichol N-acetylglucosaminyltransferase activity [GO:0004577] (molecular function) Also known as: N,N'-diacetylchitobiosylpyrophosphoryldolichol synthase activity, UDP-GlcNAc:dolichyl-pyrophosphoryl-GlcNAc GlcNAc transferase activity, UDP-N-acetyl-D-glucosamine:N-acetyl-D-glucosaminyl-diphosphodolichol N-acetyl-D-glucosaminyltransferase activity, uridine diphosphoacetylglucosamine-dolichylacetylglucosamine pyrophosphate acetylglucosaminyltransferase activity Definition: Catalysis of the reaction: UDP-N-acetyl-D-glucosamine + N-acetyl-D-glucosaminyl-diphosphodolichol = UDP + N,N''-diacetylchitobiosyldiphosphodolichol. Relationships: is a type of acetylglucosaminyltransferase activity [GO:0008375] Sources: EC:2.4.1.141